{
  "gene_symbol": "LIN7B",
  "gene": "UniProtKB:Q9HAP6",
  "gene_name": "Protein lin-7 homolog B",
  "term_label": "synapse",
  "term_id": "GO:0045202"
}